{
  "term_id": "GO:0006357",
  "term_label": "regulation of transcription by RNA polymerase II",
  "gene_name": "Transcriptional adapter 1",
  "gene_symbol": "TADA1",
  "gene": "UniProtKB:Q96BN2"
}